{
  "term_label": "positive regulation of canonical Wnt signaling pathway",
  "gene_name": "Protein FAM53B",
  "gene_symbol": "FAM53B",
  "gene": "UniProtKB:Q14153",
  "term_id": "GO:0090263"
}